{
  "term_id": "UNKNOWN:0001",
  "gene": "UniProtKB:Q9NY87",
  "gene_name": "Sperm protein associated with the nucleus on the X chromosome C",
  "term_label": "Unknown molecular function",
  "gene_symbol": "SPANXC"
}